{
  "term_label": "GTPase activator activity",
  "gene_symbol": "GIT1",
  "term_id": "GO:0005096",
  "gene_name": "ARF GTPase-activating protein GIT1",
  "gene": "UniProtKB:Q9Y2X7"
}